{
  "gene_name": "Immunoglobulin heavy variable 4-61",
  "gene_symbol": "IGHV4-61",
  "term_label": "immunoglobulin mediated immune response",
  "term_id": "GO:0016064",
  "gene": "UniProtKB:A0A0C4DH41"
}